neomycin catabolic process [GO:1901157] (biological process) Relationships: is a type of aminoglycoside antibiotic catabolic process [GO:0030649]; is a type of polyol catabolic process [GO:0046174] Also known as: neomycin breakdown, neomycin catabolism, neomycin degradation Definition: The chemical reactions and pathways resulting in the breakdown of neomycin. Sources: GOC:TermGenie, GOC:yaf, MetaCyc:PWY-7016, UniPathway:UPA00969